{
  "gene_name": "E3 ubiquitin ligase RNF121",
  "gene_symbol": "RNF121",
  "term_id": "GO:0005789",
  "term_label": "endoplasmic reticulum membrane",
  "gene": "UniProtKB:Q9H920"
}